{
  "term_label": "dolichyl-phosphate-mannose-protein mannosyltransferase activity",
  "gene_name": "Protein O-mannosyl-transferase 1",
  "term_id": "GO:0004169",
  "gene_symbol": "POMT1",
  "gene": "UniProtKB:Q9Y6A1"
}